{
  "term_label": "nucleus",
  "gene": "UniProtKB:P78414",
  "gene_name": "Iroquois-class homeodomain protein IRX-1",
  "term_id": "GO:0005634",
  "gene_symbol": "IRX1"
}